{
  "gene_name": "Sodium_hydrogen exchanger 10",
  "term_id": "GO:0015386",
  "term_label": "potassium:proton antiporter activity",
  "gene_symbol": "SLC9C1",
  "gene": "UniProtKB:Q4G0N8"
}